{
  "term_label": "protein-macromolecule adaptor activity",
  "gene_name": "RalBP1-associated Eps domain-containing protein 1",
  "gene": "UniProtKB:Q96D71",
  "term_id": "GO:0030674",
  "gene_symbol": "REPS1"
}